{
  "term_label": "axon guidance",
  "gene": "UniProtKB:Q5JYT7",
  "gene_symbol": "KIAA1755",
  "term_id": "GO:0007411",
  "gene_name": "Uncharacterized protein KIAA1755"
}